{
  "gene_name": "Phosphoenolpyruvate carboxykinase [GTP], mitochondrial",
  "gene": "UniProtKB:Q16822",
  "term_id": "GO:0032869",
  "gene_symbol": "PCK2",
  "term_label": "cellular response to insulin stimulus"
}